{
  "gene_name": "Mitogen-activated protein kinase kinase kinase 10",
  "term_label": "positive regulation of apoptotic process",
  "gene_symbol": "MAP3K10",
  "gene": "UniProtKB:Q02779",
  "term_id": "GO:0043065"
}